{
  "term_label": "cytoplasm",
  "gene_symbol": "TESK1",
  "term_id": "GO:0005737",
  "gene_name": "Dual specificity testis-specific protein kinase 1",
  "gene": "UniProtKB:Q15569"
}